{
  "gene_name": "Cytoplasmic polyadenylation element-binding protein 1",
  "gene": "UniProtKB:Q9BZB8",
  "term_id": "GO:0043022",
  "gene_symbol": "CPEB1",
  "term_label": "ribosome binding"
}